mismatch repair [GO:0006298] (biological process) References: PMID:11687886 Sources: ISBN:0198506732 Relationships: is a type of DNA repair [GO:0006281] Regulation: regulated by GO:0032423; negatively regulated by negative regulation of mismatch repair [GO:0032424]; positively regulated by positive regulation of mismatch repair [GO:0032425] Subtypes: GO:0000710, mismatch repair involved in maintenance of fidelity involved in DNA-dependent DNA replication [GO:0070716] Also known as: MMR, long patch mismatch repair system, MutS/MutL/MutH pathway, mismatch repair, MutL-like pathway Definition: A system for the correction of errors in which an incorrect base, which cannot form hydrogen bonds with the corresponding base in the parent strand, is incorporated into the daughter strand. The mismatch repair system promotes genomic fidelity by repairing base-base mismatches, insertion-deletion loops and heterologies generated during DNA replication and recombination.